limb basal epidermal cell differentiation [GO:0060889] (biological process) Relationships: is a type of epidermal cell differentiation [GO:0009913]; is a type of stem cell differentiation [GO:0048863]; is part of GO:0060887 Sources: GOC:dph, GOC:sdb_2009, GOC:tb Definition: The process in which a relatively unspecialized cell acquires specialized features of a limb epidermal basal cell. A epidermal basal cell cell is a cell that retains the ability to divide and proliferate throughout life to provide progenitor cells that can differentiate into more specialized cell of the limb epidermis.